{
  "gene": "UniProtKB:Q7Z7B8",
  "gene_name": "Beta-defensin 128",
  "gene_symbol": "DEFB128",
  "term_label": "Unknown molecular function",
  "term_id": "UNKNOWN:0001"
}